L-asparagine:sodium symporter activity [GO:0140901] (molecular function) References: PMID:21511949, PMID:28416685 Definition: Enables the transfer of a solute or solutes from one side of a membrane to the other according to the reaction: L-asparagine(out) + Na+(out) = L-asparagine(in) + Na+(in). Relationships: is a type of neutral L-amino acid:sodium symporter activity [GO:0005295]; is a type of GO:0015182; is a type of alanine:sodium symporter activity [GO:0015655] Also known as: asparagine:sodium symporter activity, sodium:L-asparagine symporter activity, sodium:asparagine symporter activity